{
  "gene": "UniProtKB:Q8IWZ6",
  "gene_symbol": "BBS7",
  "term_id": "GO:0043005",
  "gene_name": "Bardet-Biedl syndrome 7 protein",
  "term_label": "neuron projection"
}